{
  "gene": "UniProtKB:Q9P206",
  "term_label": "Unknown molecular function",
  "term_id": "UNKNOWN:0001",
  "gene_name": "Uncharacterized protein KIAA1522",
  "gene_symbol": "NHSL3"
}